{
  "term_id": "GO:0005762",
  "gene_symbol": "MRPL22",
  "gene_name": "Large ribosomal subunit protein uL22m",
  "gene": "UniProtKB:Q9NWU5",
  "term_label": "mitochondrial large ribosomal subunit"
}